glutamate-gated calcium ion channel activity [GO:0022849] (molecular function) Relationships: is a type of GO:0004970; is a type of ligand-gated calcium channel activity [GO:0099604] Sources: GOC:mtg_transport, ISBN:0815340729 Definition: Enables the transmembrane transfer of a calcium ion by a channel that opens when glutamate has been bound by the channel complex or one of its constituent parts.